{
  "gene_name": "Methyl-CpG-binding domain protein 5",
  "term_id": "GO:0005634",
  "gene_symbol": "MBD5",
  "term_label": "nucleus",
  "gene": "UniProtKB:Q9P267"
}